{
  "gene_symbol": "FES",
  "gene": "UniProtKB:P07332",
  "term_id": "GO:0005886",
  "gene_name": "Tyrosine-protein kinase Fes_Fps",
  "term_label": "plasma membrane"
}